{
  "gene_name": "Solute carrier family 2, facilitated glucose transporter member 10",
  "gene_symbol": "SLC2A10",
  "term_id": "GO:0016020",
  "gene": "UniProtKB:O95528",
  "term_label": "membrane"
}